{
  "gene_symbol": "EEF1D",
  "term_id": "GO:0005829",
  "term_label": "cytosol",
  "gene": "UniProtKB:P29692",
  "gene_name": "Elongation factor 1-delta"
}